3,4-dihydroxyphenylacetaldehyde synthase activity [GO:0106425] (molecular function) Relationships: is a type of carboxy-lyase activity [GO:0016831] Definition: Catalysis of the reaction: L-dopa + O2 + H2O + H+ = 3,4-dihydroxyphenylacetaldehyde + CO2 + NH(4)+ + H2O2. References: PMID:21283636 Sources: RHEA:55524 Also known as: DHPAA synthase